cadmium ion transmembrane transporter activity [GO:0015086] (molecular function) Definition: Enables the transfer of cadmium (Cd) ions from one side of a membrane to the other. Sources: GOC:dgf Also known as: zinc, cadmium uptake permease activity, zinc, cadmium, cobalt, nickel, lead-efflux ATPase activity Relationships: is a type of transition metal ion transmembrane transporter activity [GO:0046915]; is part of cadmium ion transmembrane transport [GO:0070574] Subtypes: GO:0008551, ABC-type cadmium transporter activity [GO:0015434]